regulation of extrinsic apoptotic signaling pathway [GO:2001236] (biological process) Definition: Any process that modulates the frequency, rate or extent of extrinsic apoptotic signaling pathway. Subtypes: regulation of extrinsic apoptotic signaling pathway via death domain receptors [GO:1902041], negative regulation of extrinsic apoptotic signaling pathway [GO:2001237], positive regulation of extrinsic apoptotic signaling pathway [GO:2001238], regulation of extrinsic apoptotic signaling pathway in absence of ligand [GO:2001239] Sources: GOC:mtg_apoptosis Relationships: is a type of regulation of apoptotic signaling pathway [GO:2001233]; regulates extrinsic apoptotic signaling pathway [GO:0097191] Also known as: regulation of extrinsic apoptotic signalling pathway, regulation of extrinsic apoptosis